muscle cell fate determination [GO:0007521] (BP) Definition: The cell fate determination process in which a cell becomes capable of differentiating autonomously into a muscle cell regardless of its environment; upon determination, the cell fate cannot be reversed. Sources: CL:0000187, GOC:go_curators Relationships: is a type of cell fate determination [GO:0001709]; is part of GO:0042693 Subtypes: cardiac muscle cell fate determination [GO:0061442], GO:0097083